negative regulation of heart rate by acetylcholine [GO:0003063] (biological process) Also known as: negative regulation of heart contraction rate by acetylcholine Sources: GOC:mtg_cardio, GOC:rl Relationships: is a type of regulation of heart rate by chemical signal [GO:0003062]; is a type of negative regulation of heart rate [GO:0010459]; BFO_0000050 regulation of systemic arterial blood pressure by acetylcholine [GO:0003068] Definition: The process in which acetylcholine released from vagus nerve endings binds to muscarinic receptors on the pacemaker cells and decreases the rate of heart muscle contraction.